{
  "term_label": "cytoplasm",
  "term_id": "GO:0005737",
  "gene_name": "Glycogen phosphorylase, liver form",
  "gene_symbol": "PYGL",
  "gene": "UniProtKB:P06737"
}